L-tryptophan aminotransferase activity [GO:0070529] (molecular function) Subtypes: GO:0050362, L-tryptophan:pyruvate aminotransferase activity [GO:0080097] Relationships: is a type of GO:0008483 Sources: GOC:mah Definition: Catalysis of the transfer of an amino group from L-tryptophan to an acceptor, usually a 2-oxo acid.